mesodermal-endodermal cell signaling [GO:0003131] (biological process) Sources: GOC:mtg_heart Definition: Any process that mediates the transfer of information from mesodermal cells to endodermal cells. Relationships: is a type of cell-cell signaling [GO:0007267] Also known as: mesodermal-endodermal cell signalling Subtypes: mesodermal-endodermal cell signaling involved in heart induction [GO:0003132]